{
  "gene": "UniProtKB:Q5BLP8",
  "term_label": "Unknown molecular function",
  "term_id": "UNKNOWN:0001",
  "gene_symbol": "NICOL1",
  "gene_name": "Neuropeptide-like protein C4orf48"
}